{
  "gene_name": "RING finger protein 222",
  "gene_symbol": "RNF222",
  "term_id": "UNKNOWN:0003",
  "term_label": "Unknown cellular component",
  "gene": "UniProtKB:A6NCQ9"
}